{
  "gene_name": "E3 ubiquitin-protein ligase ZNRF2",
  "gene": "UniProtKB:Q8NHG8",
  "term_label": "protein K48-linked ubiquitination",
  "gene_symbol": "ZNRF2",
  "term_id": "GO:0070936"
}